{
  "gene": "UniProtKB:Q16831",
  "gene_symbol": "UPP1",
  "term_label": "uridine phosphorylase activity",
  "gene_name": "Uridine phosphorylase 1",
  "term_id": "GO:0004850"
}